{
  "gene_symbol": "TRAV35",
  "term_label": "response to bacterium",
  "gene": "UniProtKB:P0DPF4",
  "gene_name": "T cell receptor alpha variable 35",
  "term_id": "GO:0009617"
}